{
  "term_id": "GO:0005856",
  "term_label": "cytoskeleton",
  "gene_name": "Rho guanine nucleotide exchange factor 2",
  "gene": "UniProtKB:Q92974",
  "gene_symbol": "ARHGEF2"
}